{
  "term_label": "cytosolic small ribosomal subunit",
  "gene_symbol": "RPS16",
  "gene_name": "Small ribosomal subunit protein uS9",
  "term_id": "GO:0022627",
  "gene": "UniProtKB:P62249"
}